neurotrophin signaling pathway [GO:0038179] (biological process) Also known as: neurotrophin receptor signaling pathway Subtypes: nerve growth factor signaling pathway [GO:0038180], neurotrophin TRK receptor signaling pathway [GO:0048011] Note: There are two classes of receptors for neurotrophins: p75 and the Trk family of tyrosine kinase receptors. Definition: The series of molecular signals initiated by neurotrophin binding to its receptor on the surface of a target cell, and ending with the regulation of a downstream cellular process, e.g. transcription. Neurotrophins are a family of secreted growth factors that induce the survival, development, and function of neurons. Relationships: is a type of cell surface receptor signaling pathway [GO:0007166]; is part of cellular response to growth factor stimulus [GO:0071363] References: PMID:17466268 Sources: GOC:bf, GOC:jc, GOC:signaling, Wikipedia:Neurotrophin